{
  "term_id": "GO:0002376",
  "gene": "UniProtKB:P14316",
  "gene_symbol": "IRF2",
  "term_label": "immune system process",
  "gene_name": "Interferon regulatory factor 2"
}